{
  "term_id": "GO:0034657",
  "gene_symbol": "RANBP9",
  "term_label": "GID complex",
  "gene": "UniProtKB:Q96S59",
  "gene_name": "Ran-binding protein 9"
}